Woronin body [GO:0140266] (cellular component) Definition: Peroxisome-derived dense-core vesicle that seals septal pores upon hyphal lysis to prevent excessive cytoplasmic loss. It is specific to several genera of filamentous ascomycetes. References: PMID:12640443, PMID:15155882, PMID:18227279, PMID:20707002, PMID:23882222 Relationships: is a type of microbody [GO:0042579]